rhombomere 7 formation [GO:0021673] (biological process) Definition: The process that gives rise to rhombomere 7. This process pertains to the initial formation of a structure from unspecified parts. Rhombomeres are transverse segments of the developing rhombencephalon. Rhombomeres are lineage restricted, express different genes from one another, and adopt different developmental fates. Rhombomeres are numbered in anterior to posterior order. Sources: GOC:cls, GOC:curators, GOC:dgh, GOC:dph, GOC:jid Relationships: is a type of rhombomere formation [GO:0021594]; is part of rhombomere 7 morphogenesis [GO:0021671]